detection of insect [GO:0009601] (biological process) Relationships: is a type of detection of other organism [GO:0098543] Also known as: perception of insect Sources: GOC:hb Definition: The series of events in which a stimulus from an insect is received and converted into a molecular signal.